{
  "term_label": "Unknown molecular function",
  "gene": "UniProtKB:O60941",
  "gene_name": "Dystrobrevin beta",
  "term_id": "UNKNOWN:0001",
  "gene_symbol": "DTNB"
}